chorionic trophoblast cell proliferation [GO:0097360] (biological process) Relationships: is a type of cell population proliferation [GO:0008283] Regulation: regulated by GO:1901382; negatively regulated by negative regulation of chorionic trophoblast cell proliferation [GO:1901383]; positively regulated by GO:1901384 Definition: The multiplication or reproduction of chorionic trophoblast cells, resulting in the expansion of their population. References: PMID:15150278 Sources: CL:0011101, GOC:BHF